{
  "gene_symbol": "JKAMP",
  "term_id": "GO:0031625",
  "gene_name": "JNK1_MAPK8-associated membrane protein",
  "gene": "UniProtKB:Q9P055",
  "term_label": "ubiquitin protein ligase binding"
}